regulation of apoptotic process involved in metanephric nephron tubule development [GO:1900217] (biological process) Definition: Any process that modulates the frequency, rate or extent of apoptotic process involved in metanephric nephron tubule development. References: PMID:17314325 Sources: GOC:TermGenie, GOC:mtg_kidney_jan10, GOC:yaf Also known as: regulation of apoptotic cell death of metanephric nephron tubule development, regulation of apoptotic process of metanephric nephron tubule development, regulation of apoptotic programmed cell death of metanephric nephron tubule development, regulation of programmed cell death by apoptosis of metanephric nephron tubule development, regulation of apoptosis of metanephric nephron tubule development, regulation of apoptotic program of metanephric nephron tubule development, regulation of type I programmed cell death of metanephric nephron tubule development, regulation of signaling (initiator) caspase activity of metanephric nephron tubule development Relationships: is a type of regulation of apoptotic process involved in development [GO:1904748]; regulates apoptotic process involved in metanephric nephron tubule development [GO:1900205] Subtypes: GO:1900218, positive regulation of apoptotic process involved in metanephric nephron tubule development [GO:1900219]